D-alanine 2-hydroxymethyltransferase activity [GO:0050413] (molecular function) Relationships: is_a hydroxymethyl-, formyl- and related transferase activity [GO:0016742] Also known as: D-alanine hydroxymethyltransferase activity, 2-methylserine hydroxymethyltransferase activity, 5,10-methylenetetrahydrofolate:D-alanine 2-hydroxymethyltransferase activity Definition: Catalysis of the reaction: 5,10-methylenetetrahydrofolate + D-alanine + H2O = (6S)-5,6,7,8-tetrahydrofolate + 2-methylserine. Sources: EC:2.1.2.7, RHEA:10064